{
  "gene": "UniProtKB:O76050",
  "term_label": "postsynaptic density",
  "gene_name": "E3 ubiquitin-protein ligase NEURL1",
  "term_id": "GO:0014069",
  "gene_symbol": "NEURL1"
}